glial cell-neuron signaling [GO:0150098] (biological process) Subtypes: GO:0036520 Definition: Cell-cell signaling that mediates the transfer of information from a glial cell to a neuron. This signaling has been shown to be mediated by various molecules, depending on which glial cells release them, and in which tissues the signaling occurs, e.g. microglial cell-derived nerve growth factor (NGF) in the retina, or microglial cell-derived superoxide ions in the cerebellum. Relationships: is a type of cell-cell signaling [GO:0007267] Also known as: glia-neuron signaling, glia-neuron signalling, glia-neurone signaling, glia-neurone signalling, glial cell- neuron signalling, glial cell-neurone signalling, glial cell-neurone singaling References: PMID:14980203, PMID:16144764, PMID:16547515, PMID:18685038, PMID:27788368, PMID:9459440 Sources: GOC:aruk, GOC:bc